{
  "gene_symbol": "FCGRT",
  "gene": "UniProtKB:P55899",
  "gene_name": "IgG receptor FcRn large subunit p51",
  "term_label": "immune response",
  "term_id": "GO:0006955"
}